{
  "term_label": "positive regulation of immune response",
  "term_id": "GO:0050778",
  "gene": "UniProtKB:P13762",
  "gene_name": "HLA class II histocompatibility antigen, DR beta 4 chain",
  "gene_symbol": "HLA-DRB4"
}